{
  "term_id": "GO:0060736",
  "gene": "UniProtKB:P07602",
  "gene_symbol": "PSAP",
  "gene_name": "Prosaposin",
  "term_label": "prostate gland growth"
}